{
  "gene_symbol": "IFNA7",
  "term_label": "adaptive immune response",
  "gene": "UniProtKB:P01567",
  "gene_name": "Interferon alpha-7",
  "term_id": "GO:0002250"
}